{
  "gene": "UniProtKB:P31937",
  "gene_name": "3-hydroxyisobutyrate dehydrogenase, mitochondrial",
  "term_label": "mitochondrion",
  "term_id": "GO:0005739",
  "gene_symbol": "HIBADH"
}